{
  "term_label": "Unknown molecular function",
  "gene_name": "Maestro heat-like repeat family member 5",
  "term_id": "UNKNOWN:0001",
  "gene_symbol": "MROH5",
  "gene": "UniProtKB:Q6ZUA9"
}